{
  "term_id": "GO:0009653",
  "term_label": "anatomical structure morphogenesis",
  "gene_name": "Forkhead box protein B1",
  "gene_symbol": "FOXB1",
  "gene": "UniProtKB:Q99853"
}